{
  "gene": "UniProtKB:Q08378",
  "term_id": "GO:0000139",
  "term_label": "Golgi membrane",
  "gene_symbol": "GOLGA3",
  "gene_name": "Golgin subfamily A member 3"
}